{
  "term_label": "Unknown molecular function",
  "gene_name": "Testis-expressed protein 45",
  "term_id": "UNKNOWN:0001",
  "gene_symbol": "TEX45",
  "gene": "UniProtKB:Q8NA69"
}